{
  "gene_name": "Ubiquitin_ISG15-conjugating enzyme E2 L6",
  "term_label": "ISG15-protein conjugation",
  "gene_symbol": "UBE2L6",
  "term_id": "GO:0032020",
  "gene": "UniProtKB:O14933"
}